{
  "gene_symbol": "SYTL4",
  "term_label": "exocytosis",
  "gene_name": "Synaptotagmin-like protein 4",
  "term_id": "GO:0006887",
  "gene": "UniProtKB:Q96C24"
}